proton-transporting two-sector ATPase complex assembly [GO:0070071] (biological process) Subtypes: proton-transporting ATP synthase complex assembly [GO:0043461], proton-transporting V-type ATPase complex assembly [GO:0070070] Sources: GOC:mah Definition: The aggregation, arrangement and bonding together of a proton-transporting two-sector ATPase complex, a large protein complex that catalyzes the synthesis or hydrolysis of ATP by a rotational mechanism, coupled to the transport of protons across a membrane. Relationships: is a type of protein-containing complex assembly [GO:0065003]